{
  "gene": "UniProtKB:Q9HBJ7",
  "gene_symbol": "USP29",
  "gene_name": "Ubiquitin carboxyl-terminal hydrolase 29",
  "term_id": "GO:0004843",
  "term_label": "cysteine-type deubiquitinase activity"
}